{
  "gene_symbol": "TRAV7",
  "gene": "UniProtKB:A0A075B6U4",
  "gene_name": "T cell receptor alpha variable 7",
  "term_label": "Unknown cellular component",
  "term_id": "UNKNOWN:0003"
}